CoA-dependent peptidyl-lysine N6-myristoyltransferase activity [GO:0140770] (molecular function) Definition: Catalysis of the reaction: L-lysyl-[protein] + tetradecanoyl-CoA = CoA + H+ + N(6)-tetradecanoyl-L-lysyl-[protein]. References: PMID:1402651 Sources: RHEA:59752 Relationships: is a type of peptidyl-lysine N6-myristoyltransferase activity [GO:0018030]